mating behavior, sex discrimination [GO:0048047] (biological process) References: PMID:12486700 Sources: GOC:jid, GOC:pr Also known as: mating behaviour, sex discrimination Relationships: is a type of mating behavior [GO:0007617] Definition: The behavior of individuals for the purpose of discriminating between the sexes, for the purpose of finding a suitable mating partner.